{
  "gene": "UniProtKB:Q86U28",
  "term_label": "iron-sulfur cluster assembly",
  "gene_name": "Iron-sulfur cluster assembly 2 homolog, mitochondrial",
  "gene_symbol": "ISCA2",
  "term_id": "GO:0016226"
}